{
  "term_id": "GO:0042981",
  "gene_symbol": "USP17L18",
  "term_label": "regulation of apoptotic process",
  "gene": "UniProtKB:D6R9N7",
  "gene_name": "Ubiquitin carboxyl-terminal hydrolase 17-like protein 18"
}